positive regulation of glial cell proliferation [GO:0060252] (biological process) Subtypes: positive regulation of Schwann cell proliferation [GO:0010625] Sources: GOC:dph, GOC:sl, GOC:tb Relationships: is a type of positive regulation of cell population proliferation [GO:0008284]; is a type of positive regulation of gliogenesis [GO:0014015]; is a type of regulation of glial cell proliferation [GO:0060251]; positively regulates GO:0014009 Definition: Any process that activates or increases the rate or extent of glial cell proliferation.